4-hydroxybutanoyl-CoA dehydratase activity [GO:0043721] (molecular function) Sources: EC:4.2.1.120 Also known as: 4-hydroxybutanoyl-CoA hydro-lyase, 4-hydroxybutyryl-CoA dehydratase activity, gamma-hydroxybutanoyl-CoA dehydratase activity, gamma-hydroxybutyryl-CoA dehydratase activity Relationships: is a type of hydro-lyase activity [GO:0016836] Definition: Catalysis of the reaction: 4-hydroxybutanoyl-CoA = vinylacetyl-CoA + H2O.